KDEL sequence binding [GO:0005046] (molecular function) Relationships: is a type of GO:0046923 Also known as: KDEL receptor activity Definition: Binding to a KDEL sequence, the C terminus tetrapeptide sequence Lys-Asp-Glu-Leu found in proteins that are to be retained in the endoplasmic reticulum. Sources: GOC:ai